{
  "term_id": "GO:0005829",
  "gene_name": "PEX5-related protein",
  "gene": "UniProtKB:Q8IYB4",
  "gene_symbol": "PEX5L",
  "term_label": "cytosol"
}